{
  "gene_name": "Delta-type opioid receptor",
  "gene": "UniProtKB:P41143",
  "gene_symbol": "OPRD1",
  "term_id": "GO:0007218",
  "term_label": "neuropeptide signaling pathway"
}